{
  "gene_name": "TRAF2 and NCK-interacting protein kinase",
  "term_label": "MAPK cascade",
  "term_id": "GO:0000165",
  "gene_symbol": "TNIK",
  "gene": "UniProtKB:Q9UKE5"
}